SsuD-SsuE complex [GO:1990200] (cellular component) Also known as: two-component alkanesulfonate monooxygenase system References: PMID:16997955 Sources: GOC:bhm Definition: A protein complex containing an alkanesulfonate monooxygenase subunit (SsuD tetramer in E.coli) and a flavin oxidoreductase subunit (SsuE dimer in E.coli). Involved in the utilization of alkanesulfonates as sulfur sources under conditions of sulfate or cysteine starvation. Relationships: is a type of protein-containing complex [GO:0032991]; is part of cytosol [GO:0005829]; has part alkanesulfonate monooxygenase complex [GO:1990201]; has part FMN reductase complex [GO:1990202]